{
  "gene_symbol": "PRDX4",
  "gene": "UniProtKB:Q13162",
  "term_label": "cell redox homeostasis",
  "term_id": "GO:0045454",
  "gene_name": "Peroxiredoxin-4"
}